{
  "gene_name": "TNFAIP3-interacting protein 2",
  "term_label": "Unknown cellular component",
  "term_id": "UNKNOWN:0003",
  "gene_symbol": "TNIP2",
  "gene": "UniProtKB:Q8NFZ5"
}